{
  "gene": "UniProtKB:O60603",
  "term_id": "GO:0038023",
  "term_label": "signaling receptor activity",
  "gene_symbol": "TLR2",
  "gene_name": "Toll-like receptor 2"
}